telomeric loop disassembly [GO:0090657] (biological process) Relationships: is a type of telomere maintenance [GO:0000723] References: PMID:22579284 Sources: GOC:BHF, GOC:BHF_telomere, GOC:nc Definition: The telomere maintenance process in which telomeric loops are disassembled to permit efficient telomere replication. Subtypes: GO:0061820 Also known as: T loop disassembly, t-loop disassembly Regulation: regulated by regulation of telomeric loop disassembly [GO:1904533]; RO_0002212 by negative regulation of telomeric loop disassembly [GO:1904534]; positively regulated by positive regulation of telomeric loop disassembly [GO:1904535]